regulation of gene silencing by regulatory ncRNA [GO:0060966] (biological process) Relationships: is a type of regulation of gene expression [GO:0010468]; regulates regulatory ncRNA-mediated gene silencing [GO:0031047] Sources: GOC:dph, GOC:tb Subtypes: GO:0010964, GO:0060967, regulation of regulatory ncRNA processing [GO:0070920], regulation of post-transcriptional gene silencing by regulatory ncRNA [GO:1900368] Definition: Any process that regulates the rate, frequency, or extent of gene silencing by RNA. Gene silencing by RNA is the process in which RNA molecules inactivate expression of target genes. Also known as: regulation of gene silencing by RNA